{
  "gene": "UniProtKB:Q9BT40",
  "term_id": "GO:0046627",
  "gene_symbol": "INPP5K",
  "gene_name": "Inositol polyphosphate 5-phosphatase K",
  "term_label": "negative regulation of insulin receptor signaling pathway"
}